S-formylglutathione hydrolase activity [GO:0018738] (molecular function) Relationships: is a type of thiolester hydrolase activity [GO:0016790] Sources: EC:3.1.2.12, RHEA:14961 Definition: Catalysis of the reaction: S-formylglutathione + H2O = formate + glutathione + H+.